{
  "gene_name": "Putative pro-MCH-like protein 2",
  "term_id": "GO:0032227",
  "gene": "UniProtKB:Q9BQD1",
  "gene_symbol": "PMCHL2",
  "term_label": "negative regulation of synaptic transmission, dopaminergic"
}